{
  "term_label": "Unknown biological process",
  "gene_name": "Cancer_testis antigen family 45 member A3",
  "term_id": "UNKNOWN:0002",
  "gene_symbol": "CT45A3",
  "gene": "UniProtKB:Q8NHU0"
}